{
  "gene_name": "Sodium-coupled neutral amino acid transporter 5",
  "gene": "UniProtKB:Q8WUX1",
  "gene_symbol": "SLC38A5",
  "term_id": "GO:0015187",
  "term_label": "glycine transmembrane transporter activity"
}